proteolysis within endoplasmic reticulum associated with antigen processing and presentation [GO:0002498] (biological process) Definition: The hydrolysis of a peptide bond or bonds within a protein by ER resident proteases contributing to antigen processing and presentation. References: PMID:15224092, PMID:15771591 Sources: GOC:add, ISBN:0781735149 Also known as: ER proteolysis associated with antigen processing and presentation, endoplasmic reticulum proteolysis associated with antigen processing and presentation, proteolysis within ER associated with antigen processing and presentation Relationships: is a type of GO:0002496